{
  "term_id": "GO:0003746",
  "gene": "UniProtKB:P57772",
  "gene_name": "Selenocysteine-specific elongation factor",
  "term_label": "translation elongation factor activity",
  "gene_symbol": "EEFSEC"
}